{
  "gene_name": "Integrator complex subunit 6-like",
  "term_id": "GO:0034472",
  "term_label": "snRNA 3'-end processing",
  "gene": "UniProtKB:Q5JSJ4",
  "gene_symbol": "INTS6L"
}